{
  "term_id": "GO:0001508",
  "gene_name": "Potassium voltage-gated channel subfamily B member 1",
  "gene": "UniProtKB:Q14721",
  "term_label": "action potential",
  "gene_symbol": "KCNB1"
}